{
  "term_id": "GO:0140566",
  "gene_symbol": "BRD1",
  "gene": "UniProtKB:O95696",
  "term_label": "histone reader activity",
  "gene_name": "Bromodomain-containing protein 1"
}